azurophil granule lumen [GO:0035578] (cellular component) Definition: The volume enclosed by the membrane of an azurophil granule, a primary lysosomal granule found in neutrophil granulocytes that contains a wide range of hydrolytic enzymes and is released into the extracellular fluid. Also known as: primary granule lumen References: PMID:17152095 Sources: GOC:bf Relationships: is a type of vacuolar lumen [GO:0005775]; is a type of GO:0034774; is part of azurophil granule [GO:0042582]